{
  "gene_symbol": "P2RY12",
  "term_label": "G protein-coupled purinergic nucleotide receptor activity",
  "term_id": "GO:0045028",
  "gene_name": "P2Y purinoceptor 12",
  "gene": "UniProtKB:Q9H244"
}